tRNA pseudouridine(31) synthase activity [GO:0160152] (MF) Relationships: is a type of tRNA pseudouridine synthase activity [GO:0106029] Definition: Catalysis of the reaction: uridine(31) in tRNA = pseudouridine(31) in tRNA. Sources: EC:5.4.99.42